{
  "term_id": "GO:0009755",
  "gene_name": "Peroxisome proliferator-activated receptor delta",
  "term_label": "hormone-mediated signaling pathway",
  "gene_symbol": "PPARD",
  "gene": "UniProtKB:Q03181"
}